chromatin silencing complex [GO:0005677] (CC) Sources: GOC:mah Subtypes: GO:0030869, eNoSc complex [GO:0061773], chromatin lock complex [GO:0061793], GO:0140283, HUSH2 complex [GO:0140286] Definition: Any protein complex that mediates changes in chromatin structure that result in transcriptional silencing. Relationships: is_a GO:0140513